{
  "term_id": "GO:0032933",
  "term_label": "SREBP signaling pathway",
  "gene_symbol": "ERLIN1",
  "gene": "UniProtKB:O75477",
  "gene_name": "Erlin-1"
}